{
  "gene_name": "Ciliogenesis and planar polarity effector 1",
  "gene": "UniProtKB:Q9H799",
  "term_id": "GO:0035869",
  "term_label": "ciliary transition zone",
  "gene_symbol": "CPLANE1"
}